peptidyl-arginine 3-dioxygenase activity [GO:0106157] (molecular function) Also known as: L-arginine 3-hydroxylase activity References: PMID:29563586 Relationships: is a type of 2-oxoglutarate-dependent dioxygenase activity [GO:0016706]; is a type of catalytic activity, acting on a protein [GO:0140096] Definition: Catalyzes the reaction: 2-oxoglutarate + [protein]-L-arginine + O2 = [protein]-(3R)-3-hydroxy-L-arginine + CO2 + succinate.